{
  "gene_name": "D(4) dopamine receptor",
  "term_id": "GO:0030425",
  "term_label": "dendrite",
  "gene": "UniProtKB:P21917",
  "gene_symbol": "DRD4"
}